regulation of mitotic cell cycle phase transition [GO:1901990] (biological process) Definition: Any process that modulates the frequency, rate or extent of mitotic cell cycle phase transition. Subtypes: regulation of exit from mitosis [GO:0007096], regulation of G2/M transition of mitotic cell cycle [GO:0010389], regulation of mitotic metaphase/anaphase transition [GO:0030071], negative regulation of mitotic cell cycle phase transition [GO:1901991], GO:1901992, GO:2000045 References: PMID:22841721 Sources: GOC:TermGenie, GOC:mtg_cell_cycle Relationships: is a type of regulation of mitotic cell cycle [GO:0007346]; is a type of GO:1901987; regulates mitotic cell cycle phase transition [GO:0044772] Also known as: mitotic cell cycle control